{
  "term_label": "chromatin DNA binding",
  "gene_name": "TOX high mobility group box family member 2",
  "gene_symbol": "TOX2",
  "term_id": "GO:0031490",
  "gene": "UniProtKB:Q96NM4"
}